{
  "gene_name": "Fanconi anemia group M protein",
  "term_id": "GO:0009378",
  "gene_symbol": "FANCM",
  "term_label": "four-way junction helicase activity",
  "gene": "UniProtKB:Q8IYD8"
}